{
  "gene": "UniProtKB:O43361",
  "term_id": "GO:0005634",
  "gene_symbol": "ZNF749",
  "term_label": "nucleus",
  "gene_name": "Zinc finger protein 749"
}